{
  "gene_name": "Prostaglandin F2 receptor negative regulator",
  "gene_symbol": "PTGFRN",
  "term_id": "UNKNOWN:0001",
  "gene": "UniProtKB:Q9P2B2",
  "term_label": "Unknown molecular function"
}